alpha6-beta4 integrin-CD151 complex [GO:0071061] (cellular component) Also known as: ITGA6-ITGB4-CD151 complex References: PMID:10811835 Definition: A protein complex that consists of an alpha6-beta4 integrin complex bound to the tetraspanin CD151. Relationships: is a type of plasma membrane protein complex [GO:0098797]